regulation of complement activation, alternative pathway [GO:0030451] (biological process) Relationships: is a type of regulation of complement activation [GO:0030449]; is a type of regulation of innate immune response [GO:0045088]; regulates GO:0006957 Definition: Any process that modulates the frequency, rate or extent of the alternative pathway of complement activation. Also known as: regulation of complement cascade, alternative pathway Sources: GOC:go_curators Subtypes: GO:0045957, positive regulation of complement activation, alternative pathway [GO:0045958]